{
  "gene_name": "Transcription initiation factor TFIID subunit 7-like",
  "term_id": "GO:0051123",
  "gene_symbol": "TAF7L",
  "term_label": "RNA polymerase II preinitiation complex assembly",
  "gene": "UniProtKB:Q5H9L4"
}